L-threonine catabolic process to acetyl-CoA [GO:0070690] (biological process) Relationships: is a type of acetyl-CoA metabolic process [GO:0006084]; is a type of GO:0006567; is a type of GO:0043605 Also known as: threonine catabolic process to acetyl-CoA, L-threonine breakdown to acetyl-CoA, L-threonine catabolism to acetyl-CoA, L-threonine degradation to acetyl-CoA Sources: GOC:bf, GOC:mah, MetaCyc:PWY-5436 Definition: The chemical reactions and pathways resulting in the breakdown of L-threonine (the L-enantiomer of 2-amino-3-hydroxybutyric acid) into glycine and acetaldehyde, with acetaldehyde being subsequently converted to acetyl-CoA.